{
  "gene": "UniProtKB:O95196",
  "gene_name": "Chondroitin sulfate proteoglycan 5",
  "term_id": "UNKNOWN:0001",
  "term_label": "Unknown molecular function",
  "gene_symbol": "CSPG5"
}